opsonin binding [GO:0001846] (molecular function) Definition: Binding to an opsonin, such as a complement component or antibody, deposited on the surface of a bacteria, virus, immune complex, or other particulate material. Relationships: is_a protein binding [GO:0005515] Note: Note that an opsonin is a blood serum protein or fragment which when deposited on the surface of a bacteria, virus, immune complex, or other particulate material acts a signal for phagocytosis to cells bearing the appropriate receptors. Not all complement components or fragments and not all antibodies have opsonic properties. Subtypes: complement component C1q complex binding [GO:0001849], complement component C3b binding [GO:0001851], GO:0001852, complement component C4b binding [GO:0001855], collectin binding [GO:0001862], pentraxin binding [GO:0001864] Sources: GOC:add, ISBN:0781735149